{
  "gene": "UniProtKB:Q9C0K1",
  "term_id": "GO:0030003",
  "gene_symbol": "SLC39A8",
  "term_label": "intracellular monoatomic cation homeostasis",
  "gene_name": "Metal cation symporter ZIP8"
}